regulation of molecular function [GO:0065009] (biological process) Sources: GOC:isa_complete Relationships: is a type of biological regulation [GO:0065007]; regulates molecular_function [GO:0003674] Definition: Any process that modulates the frequency, rate or extent of a molecular function, an elemental biological activity occurring at the molecular level, such as catalysis or binding. Also known as: regulation of a molecular function Subtypes: GO:0010469, GO:0022898, regulation of ATP-dependent activity [GO:0043462], negative regulation of molecular function [GO:0044092], positive regulation of molecular function [GO:0044093], regulation of catalytic activity [GO:0050790], GO:0051090, regulation of binding [GO:0051098]